{
  "term_id": "GO:0005125",
  "gene": "UniProtKB:P58499",
  "gene_name": "Protein FAM3B",
  "gene_symbol": "FAM3B",
  "term_label": "cytokine activity"
}